mushroom body development [GO:0016319] (BP) References: PMID:8790424 Relationships: is_a anatomical structure development [GO:0048856]; is part of brain development [GO:0007420] Definition: The process whose specific outcome is the progression of the mushroom body over time, from its formation to the mature structure. The mushroom body is composed of the prominent neuropil structures of the insect central brain, thought to be crucial for olfactory associated learning. These consist mainly of a bulbous calyx and tightly packaged arrays of thin parallel fibers of the Kenyon cells.